{
  "term_label": "Unknown molecular function",
  "gene": "UniProtKB:Q9BSF0",
  "gene_symbol": "C2orf88",
  "gene_name": "Small membrane A-kinase anchor protein",
  "term_id": "UNKNOWN:0001"
}